{
  "gene": "UniProtKB:Q9H8X9",
  "term_id": "GO:0005794",
  "gene_name": "Palmitoyltransferase ZDHHC11",
  "gene_symbol": "ZDHHC11",
  "term_label": "Golgi apparatus"
}